{
  "gene_symbol": "SNAI3",
  "gene_name": "Zinc finger protein SNAI3",
  "term_label": "RNA polymerase II cis-regulatory region sequence-specific DNA binding",
  "gene": "UniProtKB:Q3KNW1",
  "term_id": "GO:0000978"
}